{
  "term_label": "endosomal transport",
  "term_id": "GO:0016197",
  "gene_name": "Intersectin-2",
  "gene_symbol": "ITSN2",
  "gene": "UniProtKB:Q9NZM3"
}